{
  "gene": "UniProtKB:Q15040",
  "gene_name": "Josephin-1",
  "gene_symbol": "JOSD1",
  "term_id": "UNKNOWN:0003",
  "term_label": "Unknown cellular component"
}